{
  "gene_symbol": "SNX5",
  "gene": "UniProtKB:Q9Y5X3",
  "term_id": "GO:0042147",
  "gene_name": "Sorting nexin-5",
  "term_label": "retrograde transport, endosome to Golgi"
}